lysosomal proton-transporting V-type ATPase, V0 domain [GO:0046610] (CC) Relationships: is a type of vacuolar proton-transporting V-type ATPase, V0 domain [GO:0000220]; is part of lysosomal proton-transporting V-type ATPase complex [GO:0046611] Sources: GOC:mah Also known as: lysosomal hydrogen ion-transporting ATPase V0 domain Definition: The V0 domain of a proton-transporting V-type ATPase found in the lysosomal membrane.